{
  "term_label": "negative regulation of neuron apoptotic process",
  "term_id": "GO:0043524",
  "gene_symbol": "TMBIM1",
  "gene_name": "Protein lifeguard 3",
  "gene": "UniProtKB:Q969X1"
}